{
  "gene": "UniProtKB:Q04844",
  "term_label": "plasma membrane",
  "term_id": "GO:0005886",
  "gene_symbol": "CHRNE",
  "gene_name": "Acetylcholine receptor subunit epsilon"
}